{
  "gene": "UniProtKB:Q9Y2R9",
  "gene_symbol": "MRPS7",
  "term_label": "ribosome",
  "gene_name": "Small ribosomal subunit protein uS7m",
  "term_id": "GO:0005840"
}